{
  "gene": "UniProtKB:O43847",
  "gene_symbol": "NRDC",
  "term_label": "metalloendopeptidase activity",
  "gene_name": "Nardilysin",
  "term_id": "GO:0004222"
}